regulation of cell migration involved in sprouting angiogenesis [GO:0090049] (biological process) Sources: GOC:BHF, GOC:dph, GOC:rl, GOC:tb Definition: Any process that modulates the frequency, rate or extent of cell migration involved in sprouting angiogenesis. Cell migration involved in sprouting angiogenesis is the orderly movement of endothelial cells into the extracellular matrix in order to form new blood vessels contributing to the process of sprouting angiogenesis. Relationships: is a type of regulation of blood vessel endothelial cell migration [GO:0043535]; regulates cell migration involved in sprouting angiogenesis [GO:0002042] Subtypes: GO:0090050, GO:0090051